{
  "term_id": "GO:0099525",
  "term_label": "presynaptic dense core vesicle exocytosis",
  "gene": "UniProtKB:O00186",
  "gene_name": "Syntaxin-binding protein 3",
  "gene_symbol": "STXBP3"
}